{
  "term_id": "GO:0030200",
  "gene": "UniProtKB:Q8IWU5",
  "gene_name": "Extracellular sulfatase Sulf-2",
  "gene_symbol": "SULF2",
  "term_label": "heparan sulfate proteoglycan catabolic process"
}